{
  "gene_name": "Calcium-binding protein 1",
  "term_id": "GO:0007601",
  "term_label": "visual perception",
  "gene_symbol": "CABP1",
  "gene": "UniProtKB:Q9NZU7"
}